N-acetylgalactosaminoglycan deacetylase activity [GO:0047375] (MF) Also known as: N-acetyl galactosaminoglycan deacetylase activity, N-acetyl-D-galactosaminoglycan acetylhydrolase activity, Vi-polysaccharide deacetylase activity, polysaccharide deacetylase activity Relationships: is a type of deacetylase activity [GO:0019213]; is a type of carboxylic ester hydrolase activity [GO:0052689] Definition: Catalysis of the reaction: H2O + N-acetyl-D-galactosaminoglycan = acetate + D-galactosaminoglycan. Sources: EC:3.1.1.58, MetaCyc:3.1.1.58-RXN